{
  "term_label": "ubiquitin ligase complex",
  "gene_name": "E3 ubiquitin-protein ligase RNF19A",
  "gene_symbol": "RNF19A",
  "gene": "UniProtKB:Q9NV58",
  "term_id": "GO:0000151"
}